{
  "gene_name": "Diphosphoinositol polyphosphate phosphohydrolase 2",
  "term_label": "diphosphoinositol polyphosphate metabolic process",
  "gene": "UniProtKB:Q9NZJ9",
  "gene_symbol": "NUDT4",
  "term_id": "GO:0071543"
}